{
  "term_id": "GO:0051604",
  "term_label": "protein maturation",
  "gene": "UniProtKB:P49863",
  "gene_symbol": "GZMK",
  "gene_name": "Granzyme K"
}